alpha-D-ribose 1-methylphosphonate 5-triphosphate synthase complex [GO:0061694] (cellular component) References: PMID:22089136 Sources: GOC:dph Definition: A catalytic protein complex that is capable of alpha-D-ribose 1-methylphosphonate 5-triphosphate synthase activity. Note: An example of this complex is PhnI (P16687) in Escherichia coli. Relationships: is a type of transferase complex, transferring phosphorus-containing groups [GO:0061695]